{
  "term_id": "GO:0005829",
  "gene_symbol": "TPP2",
  "term_label": "cytosol",
  "gene": "UniProtKB:P29144",
  "gene_name": "Tripeptidyl-peptidase 2"
}